{
  "term_id": "GO:0051607",
  "gene": "UniProtKB:Q68D06",
  "gene_name": "Schlafen family member 13",
  "term_label": "defense response to virus",
  "gene_symbol": "SLFN13"
}